{
  "gene_symbol": "IGSF6",
  "term_id": "UNKNOWN:0001",
  "gene": "UniProtKB:O95976",
  "gene_name": "Immunoglobulin superfamily member 6",
  "term_label": "Unknown molecular function"
}